copper chaperone activity [GO:0016531] (molecular function) References: PMID:10790544, PMID:11739376 Relationships: is a type of GO:0016530; has part copper ion binding [GO:0005507] Subtypes: GO:0016532 Also known as: copper carrier activity Definition: Directly binding to and delivering copper ions to a target protein.